{
  "gene_symbol": "HLA-H",
  "gene_name": "Putative HLA class I histocompatibility antigen, alpha chain H",
  "term_id": "GO:0005615",
  "gene": "UniProtKB:P01893",
  "term_label": "extracellular space"
}